{
  "gene_name": "Calpain-10",
  "term_label": "calcium-dependent cysteine-type endopeptidase activity",
  "gene_symbol": "CAPN10",
  "term_id": "GO:0004198",
  "gene": "UniProtKB:Q9HC96"
}